{
  "term_label": "peptide modification",
  "gene_name": "Glutathione hydrolase 1 proenzyme",
  "gene_symbol": "GGT1",
  "gene": "UniProtKB:P19440",
  "term_id": "GO:0031179"
}